{
  "gene": "UniProtKB:Q6UXH1",
  "gene_name": "Protein disulfide isomerase CRELD2",
  "term_id": "UNKNOWN:0002",
  "term_label": "Unknown biological process",
  "gene_symbol": "CRELD2"
}